{
  "gene_name": "Deoxynucleotidyltransferase terminal-interacting protein 2",
  "term_id": "GO:0005730",
  "term_label": "nucleolus",
  "gene": "UniProtKB:Q5QJE6",
  "gene_symbol": "DNTTIP2"
}